{
  "gene": "UniProtKB:P01861",
  "gene_symbol": "IGHG4",
  "term_label": "complement activation, classical pathway",
  "term_id": "GO:0006958",
  "gene_name": "Immunoglobulin heavy constant gamma 4"
}